{
  "term_id": "GO:0043130",
  "gene_name": "Ubiquitin-associated protein 1",
  "gene_symbol": "UBAP1",
  "term_label": "ubiquitin binding",
  "gene": "UniProtKB:Q9NZ09"
}